{
  "gene": "UniProtKB:Q9UGC6",
  "gene_name": "Regulator of G-protein signaling 17",
  "term_label": "negative regulation of G protein-coupled receptor signaling pathway",
  "term_id": "GO:0045744",
  "gene_symbol": "RGS17"
}